positive regulation of maintenance of meiotic sister chromatid cohesion [GO:0034096] (biological process) Sources: GOC:mah, GOC:vw Definition: Any process that increases the extent to which the association between sister chromatids of a replicated chromosome is maintained during a meiotic cell cycle. Relationships: is a type of positive regulation of maintenance of sister chromatid cohesion [GO:0034093]; is a type of regulation of maintenance of meiotic sister chromatid cohesion [GO:0034094]; positively regulates GO:0034090 Subtypes: positive regulation of maintenance of meiotic sister chromatid cohesion, centromeric [GO:2000711]